{
  "gene_symbol": "PARP15",
  "term_id": "GO:0005737",
  "term_label": "cytoplasm",
  "gene": "UniProtKB:Q460N3",
  "gene_name": "Protein mono-ADP-ribosyltransferase PARP15"
}